calcium:monoatomic cation antiporter activity involved in regulation of postsynaptic cytosolic calcium ion concentration [GO:1905060] (molecular function) References: PMID:18024055 Sources: GOC:TermGenie, GO_REF:0000061 Relationships: is a type of calcium:monoatomic cation antiporter activity [GO:0015368]; is part of regulation of postsynaptic cytosolic calcium ion concentration [GO:0099566] Also known as: calcium:cation antiporter activity involved in regulation of postsynaptic cytosolic calcium ion concentration, calcium:cation antiporter activity involved in regulation of postsynaptic cytosolic calcium ion levels Definition: Any calcium:cation antiporter activity that is involved in regulation of postsynaptic cytosolic calcium ion concentration.